{
  "term_label": "endoplasmic reticulum",
  "gene": "UniProtKB:O60568",
  "gene_symbol": "PLOD3",
  "term_id": "GO:0005783",
  "gene_name": "Multifunctional procollagen lysine hydroxylase and glycosyltransferase LH3"
}